{
  "term_id": "GO:0032007",
  "gene_symbol": "TSC1",
  "term_label": "negative regulation of TOR signaling",
  "gene_name": "Hamartin",
  "gene": "UniProtKB:Q92574"
}